{
  "gene_name": "POTE ankyrin domain family member I",
  "term_id": "GO:0016020",
  "gene": "UniProtKB:P0CG38",
  "term_label": "membrane",
  "gene_symbol": "POTEI"
}